{
  "gene_symbol": "MED9",
  "gene": "UniProtKB:Q9NWA0",
  "term_label": "mediator complex",
  "term_id": "GO:0016592",
  "gene_name": "Mediator of RNA polymerase II transcription subunit 9"
}